{
  "gene": "UniProtKB:P13497",
  "gene_name": "Bone morphogenetic protein 1",
  "term_id": "GO:0004222",
  "term_label": "metalloendopeptidase activity",
  "gene_symbol": "BMP1"
}